positive regulation of cell cycle switching, mitotic to meiotic cell cycle [GO:0140648] (biological process) Definition: Any process that activates or increases the frequency, rate or extent of mitotic to meiotic cell cycle switching, the process in which a cell switches cell cycle mode from mitotic to meiotic division. References: PMID:22375066 Relationships: is a type of positive regulation of meiotic cell cycle [GO:0051446]; is a type of positive regulation of cell cycle process [GO:0090068]; is a type of regulation of cell cycle switching, mitotic to meiotic cell cycle [GO:0110044]; positively regulates cell cycle switching, mitotic to meiotic cell cycle [GO:0051728]